{
  "term_label": "Unknown biological process",
  "gene_symbol": "JPT2",
  "gene": "UniProtKB:Q9H910",
  "gene_name": "Jupiter microtubule associated homolog 2",
  "term_id": "UNKNOWN:0002"
}